{
  "term_label": "actin cytoskeleton organization",
  "term_id": "GO:0030036",
  "gene": "UniProtKB:Q9H254",
  "gene_symbol": "SPTBN4",
  "gene_name": "Spectrin beta chain, non-erythrocytic 4"
}